{
  "gene": "UniProtKB:Q9BYD9",
  "gene_name": "Actin-related protein T3",
  "term_label": "structural constituent of cytoskeleton",
  "term_id": "GO:0005200",
  "gene_symbol": "ACTRT3"
}